{
  "gene_name": "Diacylglycerol kinase zeta",
  "gene": "UniProtKB:Q13574",
  "term_label": "phosphatidic acid biosynthetic process",
  "gene_symbol": "DGKZ",
  "term_id": "GO:0006654"
}